{
  "gene_symbol": "XKR7",
  "term_label": "Unknown molecular function",
  "term_id": "UNKNOWN:0001",
  "gene_name": "XK-related protein 7",
  "gene": "UniProtKB:Q5GH72"
}